{
  "gene_name": "Ras-related protein Rab-3B",
  "gene_symbol": "RAB3B",
  "term_label": "plasma membrane",
  "term_id": "GO:0005886",
  "gene": "UniProtKB:P20337"
}